{
  "term_id": "GO:0003873",
  "gene_symbol": "PFKFB2",
  "gene_name": "6-phosphofructo-2-kinase_fructose-2,6-bisphosphatase 2",
  "gene": "UniProtKB:O60825",
  "term_label": "6-phosphofructo-2-kinase activity"
}